{
  "term_id": "GO:0016020",
  "term_label": "membrane",
  "gene": "UniProtKB:A0A1W2PS18",
  "gene_symbol": "PMIS2",
  "gene_name": "Transmembrane protein PMIS2"
}